{
  "gene": "UniProtKB:Q68DK2",
  "term_id": "GO:0032465",
  "gene_name": "Zinc finger FYVE domain-containing protein 26",
  "gene_symbol": "ZFYVE26",
  "term_label": "regulation of cytokinesis"
}